{
  "term_label": "cytoskeleton",
  "term_id": "GO:0005856",
  "gene_name": "FH1_FH2 domain-containing protein 3",
  "gene_symbol": "FHOD3",
  "gene": "UniProtKB:Q2V2M9"
}